response to bacterial lipopeptide [GO:0070339] (biological process) Definition: Any process that results in a change in state or activity of an organism (in terms of movement, secretion, enzyme production, gene expression, etc.) as a result of a bacterial lipopeptide stimulus. Subtypes: detection of bacterial lipopeptide [GO:0070340], cellular response to bacterial lipopeptide [GO:0071221], GO:0071724, GO:0071725 Relationships: is_a response to bacterial lipoprotein [GO:0032493] References: PMID:12077222 Sources: GOC:add